{
  "term_label": "negative regulation of ubiquitin-dependent protein catabolic process",
  "term_id": "GO:2000059",
  "gene": "UniProtKB:Q09019",
  "gene_name": "Dystrophia myotonica WD repeat-containing protein",
  "gene_symbol": "DMWD"
}